DH domain binding [GO:0097161] (molecular function) Definition: Binding to a DH (Dbl homology) domain of a protein. The DH domain contains three structurally conserved regions separated by more variable regions. It is composed of 11 alpha helices that are folded into a flattened, elongated alpha-helix bundle in which two of the three conserved regions, conserved region 1 (CR1) and conserved region 3 (CR3), are exposed near the centre of one surface. CR1 and CR3, together with a part of alpha-6 and the DH/PH (pleckstrin homology) junction site, constitute the Rho GTPase interacting pocket. References: PMID:12775584 Sources: GOC:yaf, InterPro:IPR000219 Relationships: is a type of GO:0019904